{
  "gene_symbol": "RAB42",
  "term_id": "GO:0003924",
  "gene_name": "Ras-related protein Rab-42",
  "gene": "UniProtKB:Q8N4Z0",
  "term_label": "GTPase activity"
}